{
  "term_id": "GO:0016339",
  "gene": "UniProtKB:Q86UP0",
  "term_label": "calcium-dependent cell-cell adhesion",
  "gene_name": "Cadherin-24",
  "gene_symbol": "CDH24"
}